{
  "term_label": "extracellular space",
  "gene": "UniProtKB:P22352",
  "gene_name": "Glutathione peroxidase 3",
  "gene_symbol": "GPX3",
  "term_id": "GO:0005615"
}